{
  "gene_name": "Thymosin beta-4",
  "gene_symbol": "TMSB4X",
  "term_id": "GO:0005829",
  "term_label": "cytosol",
  "gene": "UniProtKB:P62328"
}